{
  "gene_symbol": "WWC2",
  "gene_name": "Protein WWC2",
  "gene": "UniProtKB:Q6AWC2",
  "term_id": "GO:0035330",
  "term_label": "regulation of hippo signaling"
}